pyrimidine deoxyribonucleoside binding [GO:0032548] (molecular function) Definition: Binding to a pyrimidine deoxyribonucleoside, a compound consisting of a pyrimidine base linked to deoxyribose. Sources: GOC:mah Relationships: is a type of pyrimidine nucleoside binding [GO:0001884]; is a type of deoxyribonucleoside binding [GO:0032546]